{
  "gene": "UniProtKB:P12034",
  "gene_symbol": "FGF5",
  "term_id": "GO:0005104",
  "gene_name": "Fibroblast growth factor 5",
  "term_label": "fibroblast growth factor receptor binding"
}